{
  "term_id": "GO:0050804",
  "gene": "UniProtKB:P20783",
  "term_label": "modulation of chemical synaptic transmission",
  "gene_name": "Neurotrophin-3",
  "gene_symbol": "NTF3"
}